positive regulation of mitotic spindle organization [GO:0110028] (biological process) Subtypes: GO:0110161, positive regulation of mitotic spindle elongation (spindle phase three) [GO:0110164], positive regulation of mitotic spindle disassembly [GO:1904687] Relationships: is_a positive regulation of mitotic cell cycle [GO:0045931]; is a type of GO:0051495; is a type of regulation of mitotic spindle organization [GO:0060236]; is a type of positive regulation of cell cycle process [GO:0090068]; positively regulates mitotic spindle organization [GO:0007052] References: PMID:17576815 Sources: GOC:bhm Definition: Any process that activates or increases the frequency, rate or extent of mitotic spindle organization.